D-glucarate metabolic process [GO:0042836] (biological process) Relationships: is a type of GO:0005975; is a type of dicarboxylic acid metabolic process [GO:0043648] Definition: The chemical reactions and pathways involving D-glucarate, the D-enantiomer of glucarate. D-glucarate is derived from either D-glucose or L-gulose. Also known as: D-glucarate metabolism, saccharate metabolic process, saccharate metabolism Sources: GOC:jsg, GOC:mah, ISBN:0198506732 Subtypes: GO:0042837, D-glucarate catabolic process [GO:0042838]